cytidine deaminase activity [GO:0004126] (MF) Relationships: is a type of hydrolase activity, acting on carbon-nitrogen (but not peptide) bonds, in cyclic amidines [GO:0016814]; is a type of deaminase activity [GO:0019239] Definition: Catalysis of the reaction: cytidine + H+ + H2O = uridine + NH4 and deoxycytidine + H+ + H2O = deoxyuridine + NH4+. Also known as: (deoxy)cytidine deaminase activity, cytidine aminohydrolase activity, cytosine nucleoside deaminase activity, deoxycytidine deaminase activity Sources: EC:3.5.4.5